{
  "gene_symbol": "CNTNAP3",
  "term_label": "nervous system development",
  "gene": "UniProtKB:Q9BZ76",
  "term_id": "GO:0007399",
  "gene_name": "Contactin-associated protein-like 3"
}